negative regulation of interleukin-1 alpha production [GO:0032690] (biological process) Definition: Any process that stops, prevents, or reduces the frequency, rate, or extent of interleukin-1 alpha production. Also known as: down regulation of interleukin-1 alpha production, down-regulation of interleukin-1 alpha production, downregulation of interleukin-1 alpha production, negative regulation of IL-1 alpha production, inhibition of interleukin-1 alpha production, negative regulation of interleukin-1 alpha biosynthetic process, negative regulation of interleukin-1 alpha secretion Relationships: is a type of regulation of interleukin-1 alpha production [GO:0032650]; is a type of GO:0032692; negatively regulates interleukin-1 alpha production [GO:0032610] Sources: GOC:mah